{
  "gene": "UniProtKB:Q14BN4",
  "gene_symbol": "SLMAP",
  "gene_name": "Sarcolemmal membrane-associated protein",
  "term_id": "GO:1900825",
  "term_label": "regulation of membrane depolarization during cardiac muscle cell action potential"
}